{
  "gene": "UniProtKB:Q9UHJ9",
  "gene_name": "Post-GPI attachment to proteins factor 2",
  "gene_symbol": "PGAP2",
  "term_id": "UNKNOWN:0001",
  "term_label": "Unknown molecular function"
}